{
  "term_label": "cell fate specification",
  "gene_symbol": "TBX22",
  "gene": "UniProtKB:Q9Y458",
  "gene_name": "T-box transcription factor TBX22",
  "term_id": "GO:0001708"
}